chitosan binding [GO:2001080] (molecular function) Definition: Binding to chitosan. Sources: GOC:mengo_curators Relationships: is a type of cation binding [GO:0043169]; is a type of carbohydrate derivative binding [GO:0097367]